{
  "term_id": "GO:0007631",
  "gene_name": "Prolactin-releasing peptide",
  "term_label": "feeding behavior",
  "gene": "UniProtKB:P81277",
  "gene_symbol": "PRLH"
}